regulation of CD8-positive, alpha-beta T cell activation [GO:2001185] (BP) Relationships: is a type of regulation of alpha-beta T cell activation [GO:0046634]; regulates CD8-positive, alpha-beta T cell activation [GO:0036037] Subtypes: GO:0043376, regulation of CD8-positive, alpha-beta T cell proliferation [GO:2000564], negative regulation of CD8-positive, alpha-beta T cell activation [GO:2001186], GO:2001187 Definition: Any process that modulates the frequency, rate or extent of CD8-positive, alpha-beta T cell activation. Sources: GOC:obol